{
  "term_label": "Unknown molecular function",
  "gene_name": "Meiosis initiator protein",
  "gene_symbol": "MEIOSIN",
  "gene": "UniProtKB:C9JSJ3",
  "term_id": "UNKNOWN:0001"
}